bilirubin oxidase activity [GO:0047705] (molecular function) Definition: Catalysis of the reaction: 2 bilirubin + O2 = 2 biliverdin + 2 H2O. Sources: EC:1.3.3.5, RHEA:20980 Also known as: bilirubin oxidase M-1, bilirubin:oxygen oxidoreductase activity Relationships: is a type of oxidoreductase activity, acting on the CH-CH group of donors, oxygen as acceptor [GO:0016634]